{
  "gene": "UniProtKB:Q9UMX6",
  "term_id": "GO:0009966",
  "gene_symbol": "GUCA1B",
  "term_label": "regulation of signal transduction",
  "gene_name": "Guanylyl cyclase-activating protein 2"
}